{
  "gene_name": "Protein FAM221B",
  "term_label": "Unknown biological process",
  "term_id": "UNKNOWN:0002",
  "gene": "UniProtKB:A6H8Z2",
  "gene_symbol": "FAM221B"
}